{
  "gene_name": "Vesicular glutamate transporter 1",
  "gene_symbol": "SLC17A7",
  "term_label": "excitatory synapse",
  "gene": "UniProtKB:Q9P2U7",
  "term_id": "GO:0060076"
}